{
  "gene_symbol": "ERVPABLB-1",
  "gene_name": "Endogenous retrovirus group PABLB member 1 Env polyprotein",
  "gene": "UniProtKB:P60509",
  "term_id": "UNKNOWN:0001",
  "term_label": "Unknown molecular function"
}